3-beta-hydroxysteroid dehydrogenase [NAD(P)+]/C4-decarboxylase activity [GO:0000252] (molecular function) Relationships: is a type of steroid dehydrogenase activity, acting on the CH-OH group of donors, NAD or NADP as acceptor [GO:0033764] Definition: Catalysis of the reaction: a 3-beta-hydroxysteroid-4-alpha-carboxylate + NADP+ = a 3-oxosteroid + CO2 + NADPH. Also known as: 3beta-hydroxy-4beta-methyl-5alpha-cholest-7-ene-4alpha-carboxylate:NAD(P)+ 3-oxidoreductase (decarboxylating), C-3 sterol dehydrogenase (C-4 sterol decarboxylase) activity, 3beta-hydroxy-4alpha-methylcholestenecarboxylate 3-dehydrogenase (decarboxylating), 3beta-hydroxy-4beta-methylcholestenecarboxylate 3-dehydrogenase (decarboxylating), 3beta-hydroxy-4beta-methylcholestenoate dehydrogenase activity, C-3 sterol dehydrogenase (C-4 decarboxylase) activity, C-3 sterol dehydrogenase activity, sterol 4alpha-carboxylic decarboxylase activity, sterol-4-carboxylate 3-dehydrogenase (decarboxylating) activity, sterol-4alpha-carboxylate 3-dehydrogenase (decarboxylating) References: PMID:9811880 Sources: EC:1.1.1.170 Subtypes: GO:0102175